{
  "term_id": "GO:0004984",
  "gene_symbol": "OR2AE1",
  "gene": "UniProtKB:Q8NHA4",
  "term_label": "olfactory receptor activity",
  "gene_name": "Olfactory receptor 2AE1"
}